{
  "term_label": "DNA binding",
  "gene": "UniProtKB:Q86W54",
  "term_id": "GO:0003677",
  "gene_symbol": "SPATA24",
  "gene_name": "Spermatogenesis-associated protein 24"
}